{
  "gene": "UniProtKB:Q01892",
  "gene_name": "Transcription factor Spi-B",
  "term_id": "GO:0030154",
  "term_label": "cell differentiation",
  "gene_symbol": "SPIB"
}